iodide channel activity [GO:0160081] (molecular function) Relationships: is_a monoatomic anion channel activity [GO:0005253]; is a type of iodide transmembrane transporter activity [GO:0015111] References: PMID:34910516 Definition: Enables the energy-independent facilitated diffusion of iodide through a transmembrane aqueous pore or channel.